{
  "gene": "UniProtKB:O75486",
  "term_id": "GO:0003713",
  "term_label": "transcription coactivator activity",
  "gene_symbol": "SUPT3H",
  "gene_name": "Transcription initiation protein SPT3 homolog"
}